{
  "gene_symbol": "AMZ2",
  "gene": "UniProtKB:Q86W34",
  "gene_name": "Archaemetzincin-2",
  "term_id": "UNKNOWN:0003",
  "term_label": "Unknown cellular component"
}